EGF-domain serine xylosyltransferase activity [GO:0140562] (molecular function) Sources: RHEA:62016 Definition: Catalyses the reaction: UDP-alpha-D-xylose + [protein with EGF-like domain]-L-serine = UDP + [protein with EGF-like domain]-3-O-(beta-D-xylosyl)-L-serine. Relationships: is a type of UDP-xylosyltransferase activity [GO:0035252]